deoxyuridine biosynthetic process [GO:0046097] (biological process) Also known as: deoxyuridine anabolism, deoxyuridine biosynthesis, deoxyuridine formation, deoxyuridine synthesis Relationships: is a type of deoxyuridine metabolic process [GO:0046096]; is_a GO:0046126 Definition: The chemical reactions and pathways resulting in the formation of deoxyuridine, 2-deoxyribosyluracil, one of the four major nucleosides of DNA. Sources: GOC:go_curators